{
  "gene_name": "Leukocyte immunoglobulin-like receptor subfamily A member 5",
  "gene": "UniProtKB:A6NI73",
  "term_id": "GO:0032396",
  "term_label": "inhibitory MHC class I receptor activity",
  "gene_symbol": "LILRA5"
}